11-deoxycorticosterone binding [GO:1903878] (molecular function) Definition: Binding to 11-deoxycorticosterone. Relationships: is a type of alcohol binding [GO:0043178]; is a type of steroid hormone binding [GO:1990239] References: PMID:10802282 Sources: GOC:TermGenie, GOC:mr, GO_REF:0000067